{
  "term_id": "UNKNOWN:0001",
  "term_label": "Unknown molecular function",
  "gene": "UniProtKB:O14727",
  "gene_name": "Apoptotic protease-activating factor 1",
  "gene_symbol": "APAF1"
}